{
  "term_id": "GO:0006302",
  "gene": "UniProtKB:Q9NXR7",
  "gene_symbol": "BABAM2",
  "gene_name": "BRISC and BRCA1-A complex member 2",
  "term_label": "double-strand break repair"
}